{
  "term_id": "GO:0035194",
  "term_label": "regulatory ncRNA-mediated post-transcriptional gene silencing",
  "gene": "UniProtKB:P42694",
  "gene_name": "Probable helicase with zinc finger domain",
  "gene_symbol": "HELZ"
}